{
  "gene_symbol": "DNAJB6",
  "gene": "UniProtKB:O75190",
  "gene_name": "DnaJ homolog subfamily B member 6",
  "term_label": "nucleus",
  "term_id": "GO:0005634"
}